{
  "gene_name": "Serpin H1",
  "gene_symbol": "SERPINH1",
  "term_id": "GO:0030199",
  "gene": "UniProtKB:P50454",
  "term_label": "collagen fibril organization"
}